{
  "term_id": "GO:0005658",
  "gene_name": "DNA polymerase alpha catalytic subunit",
  "gene": "UniProtKB:P09884",
  "gene_symbol": "POLA1",
  "term_label": "alpha DNA polymerase:primase complex"
}